{
  "gene_symbol": "ASRGL1",
  "gene": "UniProtKB:Q7L266",
  "term_id": "GO:0005737",
  "gene_name": "Isoaspartyl peptidase_L-asparaginase",
  "term_label": "cytoplasm"
}